{
  "term_id": "GO:0008812",
  "gene_symbol": "CHDH",
  "gene_name": "Choline dehydrogenase, mitochondrial",
  "term_label": "choline dehydrogenase activity",
  "gene": "UniProtKB:Q8NE62"
}